{
  "term_id": "GO:0032496",
  "gene_symbol": "PALM3",
  "term_label": "response to lipopolysaccharide",
  "gene_name": "Paralemmin-3",
  "gene": "UniProtKB:A6NDB9"
}